{
  "term_label": "heterophilic cell-cell adhesion",
  "term_id": "GO:0007157",
  "gene": "UniProtKB:Q14982",
  "gene_symbol": "OPCML",
  "gene_name": "Opioid-binding protein_cell adhesion molecule"
}